{
  "term_id": "GO:1990841",
  "gene_name": "Tumor protein 63",
  "gene": "UniProtKB:Q9H3D4",
  "term_label": "promoter-specific chromatin binding",
  "gene_symbol": "TP63"
}